{
  "gene_symbol": "PRMT8",
  "term_id": "GO:0035241",
  "gene_name": "Protein arginine N-methyltransferase 8",
  "term_label": "protein-arginine omega-N monomethyltransferase activity",
  "gene": "UniProtKB:Q9NR22"
}